{
  "gene": "UniProtKB:B3KU38",
  "term_label": "cell junction",
  "gene_name": "IQCJ-SCHIP1 readthrough transcript protein",
  "gene_symbol": "IQCJ-SCHIP1",
  "term_id": "GO:0030054"
}